gynoecium development [GO:0048467] (biological process) Relationships: is a type of GO:0048438 Sources: GOC:go_curators, PO:0008062 Definition: The process whose specific outcome is the progression of the gynoecium over time, from its formation to the mature structure. The gynoecium is the collective name for the carpels of a flower. Also known as: pistil development Subtypes: transmitting tissue development [GO:0010500]